{
  "gene_symbol": "SLC7A5P1",
  "term_id": "UNKNOWN:0003",
  "gene_name": "Putative L-type amino acid transporter 1-like protein MLAS",
  "gene": "UniProtKB:Q8MH63",
  "term_label": "Unknown cellular component"
}